{
  "term_id": "GO:0015137",
  "gene": "UniProtKB:Q8TD22",
  "gene_symbol": "SFXN5",
  "gene_name": "Sideroflexin-5",
  "term_label": "citrate transmembrane transporter activity"
}